{
  "gene": "UniProtKB:Q8N5S9",
  "term_id": "GO:0005516",
  "gene_name": "Calcium_calmodulin-dependent protein kinase kinase 1",
  "gene_symbol": "CAMKK1",
  "term_label": "calmodulin binding"
}